vestibulocochlear nerve development [GO:0021562] (biological process) Definition: The process whose specific outcome is the progression of the vestibulocochlear nerve over time, from its formation to the mature structure. This sensory nerve innervates the membranous labyrinth of the inner ear. The vestibular branch innervates the vestibular apparatus that senses head position changes relative to gravity. The auditory branch innervates the cochlear duct, which is connected to the three bony ossicles which transduce sound waves into fluid movement in the cochlea. Also known as: CN VIII development, acoustic nerve development, cranial nerve 8 development, cranial nerve VIII development Sources: GOC:cls, GOC:dgh, GOC:dph, GOC:jid, GO_REF:0000021 Relationships: is a type of cranial nerve development [GO:0021545]